{
  "gene_symbol": "MTM1",
  "gene": "UniProtKB:Q13496",
  "term_id": "GO:0016020",
  "gene_name": "Myotubularin",
  "term_label": "membrane"
}